{
  "term_id": "GO:0010975",
  "gene_symbol": "KIF26A",
  "gene_name": "Kinesin-like protein KIF26A",
  "term_label": "regulation of neuron projection development",
  "gene": "UniProtKB:Q9ULI4"
}